{
  "gene_name": "Complement C4-A",
  "term_id": "GO:0006956",
  "term_label": "complement activation",
  "gene": "UniProtKB:P0C0L4",
  "gene_symbol": "C4A"
}